{
  "term_id": "UNKNOWN:0002",
  "gene_symbol": "COLGALT2",
  "gene": "UniProtKB:Q8IYK4",
  "gene_name": "Procollagen galactosyltransferase 2",
  "term_label": "Unknown biological process"
}